P2Y6 nucleotide receptor binding [GO:0031816] (molecular function) Also known as: P2Y6 nucleotide receptor ligand Definition: Binding to a P2Y6 nucleotide receptor. Sources: GOC:mah, GOC:nln Relationships: is a type of G protein-coupled nucleotide receptor binding [GO:0031811]